{
  "gene_name": "Golgi-associated kinase 1B",
  "term_label": "Unknown biological process",
  "gene_symbol": "GASK1B",
  "gene": "UniProtKB:Q6UWH4",
  "term_id": "UNKNOWN:0002"
}